{
  "term_id": "UNKNOWN:0002",
  "gene": "UniProtKB:Q96FQ6",
  "gene_name": "Protein S100-A16",
  "term_label": "Unknown biological process",
  "gene_symbol": "S100A16"
}